{
  "gene_symbol": "ELOVL1",
  "term_id": "GO:0005789",
  "term_label": "endoplasmic reticulum membrane",
  "gene_name": "Elongation of very long chain fatty acids protein 1",
  "gene": "UniProtKB:Q9BW60"
}